{
  "gene": "UniProtKB:Q8N4Q1",
  "term_label": "mitochondrial intermembrane space",
  "gene_symbol": "CHCHD4",
  "term_id": "GO:0005758",
  "gene_name": "Mitochondrial intermembrane space import and assembly protein 40"
}